{
  "gene_name": "Mitochondrial amidoxime reducing component 2",
  "gene": "UniProtKB:Q969Z3",
  "gene_symbol": "MTARC2",
  "term_label": "nitrate reductase activity",
  "term_id": "GO:0008940"
}